{
  "term_label": "Unknown biological process",
  "gene": "UniProtKB:Q6P161",
  "gene_symbol": "MRPL54",
  "term_id": "UNKNOWN:0002",
  "gene_name": "Large ribosomal subunit protein mL54"
}